{
  "gene_symbol": "SLC5A7",
  "term_id": "GO:0007274",
  "term_label": "neuromuscular synaptic transmission",
  "gene": "UniProtKB:Q9GZV3",
  "gene_name": "High affinity choline transporter 1"
}